{
  "gene_symbol": "FLT3",
  "gene_name": "Receptor-type tyrosine-protein kinase FLT3",
  "term_label": "cytokine-mediated signaling pathway",
  "gene": "UniProtKB:P36888",
  "term_id": "GO:0019221"
}